{
  "gene": "UniProtKB:Q9UK17",
  "term_label": "neuronal cell body",
  "gene_name": "Potassium voltage-gated channel subfamily D member 3",
  "gene_symbol": "KCND3",
  "term_id": "GO:0043025"
}